{
  "gene": "UniProtKB:Q14774",
  "gene_name": "H2.0-like homeobox protein",
  "term_label": "Unknown biological process",
  "gene_symbol": "HLX",
  "term_id": "UNKNOWN:0002"
}